{
  "gene_symbol": "NXN",
  "gene_name": "Nucleoredoxin",
  "term_label": "negative regulation of protein ubiquitination",
  "term_id": "GO:0031397",
  "gene": "UniProtKB:Q6DKJ4"
}